{
  "term_id": "GO:0071011",
  "term_label": "precatalytic spliceosome",
  "gene": "UniProtKB:Q7RTV0",
  "gene_symbol": "PHF5A",
  "gene_name": "PHD finger-like domain-containing protein 5A"
}